{
  "gene_name": "Teneurin-1",
  "gene": "UniProtKB:Q9UKZ4",
  "gene_symbol": "TENM1",
  "term_id": "GO:0048666",
  "term_label": "neuron development"
}